{
  "gene_symbol": "PSMB7",
  "term_id": "GO:0019774",
  "gene_name": "Proteasome subunit beta type-7",
  "term_label": "proteasome core complex, beta-subunit complex",
  "gene": "UniProtKB:Q99436"
}